{
  "term_label": "olfactory receptor activity",
  "term_id": "GO:0004984",
  "gene_symbol": "OR8H2",
  "gene": "UniProtKB:Q8N162",
  "gene_name": "Olfactory receptor 8H2"
}